{
  "term_label": "phenylpyruvate tautomerase activity",
  "term_id": "GO:0050178",
  "gene_name": "D-dopachrome decarboxylase-like protein",
  "gene_symbol": "DDTL",
  "gene": "UniProtKB:A6NHG4"
}